{
  "gene_symbol": "IRAK4",
  "term_id": "GO:0043123",
  "term_label": "positive regulation of canonical NF-kappaB signal transduction",
  "gene_name": "Interleukin-1 receptor-associated kinase 4",
  "gene": "UniProtKB:Q9NWZ3"
}